ligase inhibitor activity [GO:0055104] (molecular function) Relationships: is a type of enzyme inhibitor activity [GO:0004857]; is a type of ligase regulator activity [GO:0055103]; negatively regulates ligase activity [GO:0016874] Definition: Binds to and stops, prevents or reduces the activity of a ligase. Sources: GOC:BHF, GOC:rl